{
  "term_label": "embryonic pattern specification",
  "term_id": "GO:0009880",
  "gene_name": "Homeobox protein Meis1",
  "gene": "UniProtKB:O00470",
  "gene_symbol": "MEIS1"
}